peroxisomal matrix [GO:0005782] (cellular component) Also known as: peroxisomal lumen Relationships: is a type of GO:0031907; BFO_0000050 GO:0005777 Definition: The volume contained within the membranes of a peroxisome; in many cells the matrix contains a crystalloid core largely composed of urate oxidase. Sources: GOC:curators, ISBN:0815316194 Subtypes: glyoxysomal lumen [GO:0031908], GO:0034468